Edg-7 lysophosphatidic acid receptor binding [GO:0031760] (molecular function) Definition: Binding to an Edg-7 lysophosphatidic acid receptor. Also known as: LPA3 receptor binding, Edg-7 lysophosphatidic acid receptor ligand Relationships: is a type of endothelial differentiation G protein-coupled receptor binding [GO:0031753] Sources: GOC:mah, GOC:nln